regulation of brain-derived neurotrophic factor receptor signaling pathway [GO:0031548] (biological process) Definition: Any process that modulates the frequency, rate or extent of signaling via the brain-derived neurotrophic factor receptor signaling pathway. Subtypes: negative regulation of brain-derived neurotrophic factor receptor signaling pathway [GO:0031549], positive regulation of brain-derived neurotrophic factor receptor signaling pathway [GO:0031550] Sources: GOC:mah Relationships: is a type of regulation of signal transduction [GO:0009966]; regulates brain-derived neurotrophic factor receptor signaling pathway [GO:0031547] Also known as: regulation of BDNF receptor signaling pathway, regulation of BDNF receptor signalling pathway, regulation of brain-derived neurotrophic factor receptor signalling pathway